{
  "gene_symbol": "ERFL",
  "term_label": "cell differentiation",
  "gene_name": "ETS domain-containing transcription factor ERF-like",
  "gene": "UniProtKB:A0A1W2PQ73",
  "term_id": "GO:0030154"
}